{
  "term_label": "plasma lipoprotein particle clearance",
  "gene_name": "Scavenger receptor class B member 1",
  "gene": "UniProtKB:Q8WTV0",
  "gene_symbol": "SCARB1",
  "term_id": "GO:0034381"
}